{
  "term_id": "GO:0008076",
  "gene_name": "Potassium voltage-gated channel subfamily KQT member 3",
  "gene_symbol": "KCNQ3",
  "term_label": "voltage-gated potassium channel complex",
  "gene": "UniProtKB:O43525"
}